{
  "gene_symbol": "ALDOB",
  "term_label": "glycolytic process",
  "term_id": "GO:0006096",
  "gene": "UniProtKB:P05062",
  "gene_name": "Fructose-bisphosphate aldolase B"
}